{
  "gene": "UniProtKB:P0DMQ9",
  "gene_symbol": "C8orf89",
  "term_label": "Unknown cellular component",
  "term_id": "UNKNOWN:0003",
  "gene_name": "Putative uncharacterized protein C8orf89"
}